{
  "gene": "UniProtKB:P60321",
  "gene_name": "Nanos homolog 2",
  "term_id": "GO:0017148",
  "gene_symbol": "NANOS2",
  "term_label": "negative regulation of translation"
}